alpha-zingiberene synthase activity [GO:0102884] (molecular function) Definition: Catalysis of the reaction: 2-trans,6-trans-farnesyl diphosphate = zingiberene + diphosphoric acid. Relationships: is a type of carbon-oxygen lyase activity, acting on phosphates [GO:0016838] Sources: EC:4.2.3.65, GOC:pz